thioester transport [GO:1901337] (biological process) Relationships: is a type of GO:0072348 Subtypes: fatty-acyl-CoA transport [GO:0015916] Sources: GOC:TermGenie Definition: The directed movement of a thioester into, out of or within a cell, or between cells, by means of some agent such as a transporter or pore.